{
  "gene_symbol": "ZDHHC4",
  "gene_name": "Palmitoyltransferase ZDHHC4",
  "term_label": "protein-cysteine S-palmitoyltransferase activity",
  "term_id": "GO:0019706",
  "gene": "UniProtKB:Q9NPG8"
}